chitinase activity [GO:0004568] (molecular function) Subtypes: endochitinase activity [GO:0008843], exochitinase activity [GO:0035885] References: PMID:11468293 Sources: GOC:bf, GOC:kah, GOC:pde Relationships: is_a hydrolase activity, hydrolyzing O-glycosyl compounds [GO:0004553] Definition: Catalysis of the hydrolysis of (1->4)-beta linkages of N-acetyl-D-glucosamine (GlcNAc) polymers of chitin and chitodextrins.